positive regulation of quinolinate biosynthetic process [GO:1904986] (biological process) Relationships: is a type of positive regulation of biosynthetic process [GO:0009891]; is a type of positive regulation of small molecule metabolic process [GO:0062013]; is a type of regulation of quinolinate biosynthetic process [GO:1904984]; positively regulates quinolinate biosynthetic process [GO:0019805] Definition: Any process that activates or increases the frequency, rate or extent of quinolinate biosynthetic process. Also known as: positive regulation of quinolinate anabolism, positive regulation of quinolinate biosynthesis, positive regulation of quinolinate formation, positive regulation of quinolinate synthesis, up regulation of quinolinate anabolism, up regulation of quinolinate biosynthesis, up regulation of quinolinate biosynthetic process, up regulation of quinolinate formation, up regulation of quinolinate synthesis, up-regulation of quinolinate anabolism, up-regulation of quinolinate biosynthesis, up-regulation of quinolinate biosynthetic process, up-regulation of quinolinate formation, up-regulation of quinolinate synthesis, upregulation of quinolinate anabolism, upregulation of quinolinate biosynthesis, upregulation of quinolinate biosynthetic process, upregulation of quinolinate formation, upregulation of quinolinate synthesis, activation of quinolinate anabolism, activation of quinolinate biosynthesis, activation of quinolinate biosynthetic process, activation of quinolinate formation, activation of quinolinate synthesis Sources: GOC:PARL, GOC:TermGenie, GOC:bf, GO_REF:0000058